cellular response to magnetism [GO:0071259] (biological process) Sources: GOC:mah Relationships: is a type of response to magnetism [GO:0071000]; is a type of cellular response to abiotic stimulus [GO:0071214] Also known as: cellular response to magnetic stimulus Definition: Any process that results in a change in state or activity of a cell (in terms of movement, secretion, enzyme production, gene expression, etc.) as a result of a magnetic stimulus.